{
  "term_id": "UNKNOWN:0001",
  "gene_symbol": "TMEM237",
  "term_label": "Unknown molecular function",
  "gene_name": "Transmembrane protein 237",
  "gene": "UniProtKB:Q96Q45"
}